{
  "gene_symbol": "CCDC88B",
  "gene": "UniProtKB:A6NC98",
  "term_id": "GO:0008017",
  "gene_name": "Coiled-coil domain-containing protein 88B",
  "term_label": "microtubule binding"
}